{
  "gene_name": "Kelch repeat and BTB domain-containing protein 4",
  "gene_symbol": "KBTBD4",
  "term_label": "Unknown biological process",
  "term_id": "UNKNOWN:0002",
  "gene": "UniProtKB:Q9NVX7"
}